{
  "term_id": "UNKNOWN:0002",
  "gene_name": "Uteroglobin",
  "term_label": "Unknown biological process",
  "gene_symbol": "SCGB1A1",
  "gene": "UniProtKB:P11684"
}